dorsal closure, leading edge cell differentiation [GO:0046663] (biological process) Definition: The process in which a relatively unspecialized cell acquires specialized features of a leading edge cell, the dorsal-most cells of the epidermis that migrates during dorsal closure. References: PMID:12147138 Sources: GOC:ai Relationships: is a type of leading edge cell differentiation [GO:0035026]; is part of initiation of dorsal closure [GO:0007392]